{
  "gene_name": "Oocyte-secreted protein 4B",
  "gene": "UniProtKB:A0A2R8Y4Y8",
  "term_id": "UNKNOWN:0002",
  "gene_symbol": "OOSP4B",
  "term_label": "Unknown biological process"
}